cell division site [GO:0032153] (CC) Note: Note that this term refers to the future site of division in a cell that has not yet divided. Definition: The eventual plane of cell division (also known as cell cleavage or cytokinesis) in a dividing cell. In Eukaryotes, the cleavage apparatus, composed of septin structures and the actomyosin contractile ring, forms along this plane, and the mitotic, or meiotic, spindle is aligned perpendicular to the division plane. In bacteria, the cell division site is generally located at mid-cell and is the site at which the cytoskeletal structure, the Z-ring, assembles. Relationships: is a type of cellular anatomical structure [GO:0110165] References: PMID:12101122, PMID:15380095, PMID:16983191, PMID:18165305 Sources: GOC:bf, GOC:imk, GOC:krc, GOC:ns Also known as: cell division plane